{
  "gene_symbol": "TBC1D21",
  "term_label": "cytoplasmic vesicle",
  "gene": "UniProtKB:Q8IYX1",
  "gene_name": "TBC1 domain family member 21",
  "term_id": "GO:0031410"
}